{
  "gene_symbol": "NACAD",
  "term_label": "unfolded protein binding",
  "gene": "UniProtKB:O15069",
  "term_id": "GO:0051082",
  "gene_name": "NAC-alpha domain-containing protein 1"
}